{
  "gene": "UniProtKB:P19397",
  "gene_name": "Leukocyte surface antigen CD53",
  "gene_symbol": "CD53",
  "term_label": "Unknown molecular function",
  "term_id": "UNKNOWN:0001"
}